{
  "term_label": "regulation of lamellipodium morphogenesis",
  "gene_symbol": "VIL1",
  "gene_name": "Villin-1",
  "gene": "UniProtKB:P09327",
  "term_id": "GO:2000392"
}